{
  "gene_symbol": "BAIAP3",
  "gene": "UniProtKB:O94812",
  "term_label": "late endosome membrane",
  "term_id": "GO:0031902",
  "gene_name": "BAI1-associated protein 3"
}